{
  "term_label": "retinoic acid receptor signaling pathway",
  "gene_name": "Retinoic acid receptor gamma",
  "term_id": "GO:0048384",
  "gene": "UniProtKB:P13631",
  "gene_symbol": "RARG"
}